{
  "gene": "UniProtKB:Q8N8Z3",
  "gene_symbol": "DIP2C-AS1",
  "term_id": "UNKNOWN:0003",
  "term_label": "Unknown cellular component",
  "gene_name": "Putative uncharacterized protein DIP2C-AS1"
}